{
  "term_id": "UNKNOWN:0002",
  "gene_symbol": "NPIPB7",
  "gene_name": "Nuclear pore complex-interacting protein family member B7",
  "term_label": "Unknown biological process",
  "gene": "UniProtKB:O75200"
}